{
  "gene_symbol": "ZNF589",
  "term_id": "GO:0005634",
  "gene_name": "Zinc finger protein 589",
  "term_label": "nucleus",
  "gene": "UniProtKB:Q86UQ0"
}